{
  "gene_name": "Ubiquitin carboxyl-terminal hydrolase 1",
  "gene": "UniProtKB:O94782",
  "term_label": "cysteine-type deubiquitinase activity",
  "gene_symbol": "USP1",
  "term_id": "GO:0004843"
}